{
  "gene_symbol": "F2RL1",
  "gene_name": "Proteinase-activated receptor 2",
  "gene": "UniProtKB:P55085",
  "term_label": "positive regulation of Rho protein signal transduction",
  "term_id": "GO:0035025"
}